{
  "gene": "UniProtKB:Q9BSI4",
  "gene_symbol": "TINF2",
  "gene_name": "TERF1-interacting nuclear factor 2",
  "term_id": "GO:0070187",
  "term_label": "shelterin complex"
}